{
  "term_label": "regulation of transcription by RNA polymerase II",
  "term_id": "GO:0006357",
  "gene": "UniProtKB:Q86YE8",
  "gene_symbol": "ZNF573",
  "gene_name": "Zinc finger protein 573"
}